RNA polymerase II CTD heptapeptide repeat S7 kinase activity [GO:0140837] (molecular function) References: PMID:28248323 Relationships: is a type of RNA polymerase II CTD heptapeptide repeat kinase activity [GO:0008353] Definition: Catalysis of the reaction: ATP + RNA polymerase II large subunit CTD heptapeptide repeat (consensus YSPTSPS) = ADP + H+ + RNA polymerase II large subunit phosphoserine (position 7). Also known as: RNA polymerase II C-terminal domain S7 kinase activity